{
  "term_label": "Unknown cellular component",
  "gene": "UniProtKB:Q9UJS0",
  "gene_name": "Electrogenic aspartate_glutamate antiporter SLC25A13, mitochondrial",
  "gene_symbol": "SLC25A13",
  "term_id": "UNKNOWN:0003"
}